{
  "term_label": "cilium movement",
  "gene": "UniProtKB:Q6P9G0",
  "gene_symbol": "CYB5D1",
  "term_id": "GO:0003341",
  "gene_name": "Cytochrome b5 domain-containing protein 1"
}